{
  "gene_name": "Vasopressin-neurophysin 2-copeptin",
  "term_label": "secretory granule",
  "term_id": "GO:0030141",
  "gene_symbol": "AVP",
  "gene": "UniProtKB:P01185"
}